coenzyme F420-2 alpha-glutamyl ligase activity [GO:0043774] (molecular function) Definition: Catalysis of the reaction: coenzyme F420-2 + L-glutamate + GTP = coenzyme F420-3 + GDP + orthophosphate. Also known as: F420-2 alpha-glutamyl ligase activity Relationships: is a type of acid-amino acid ligase activity [GO:0016881] References: PMID:12909715